{
  "gene_symbol": "FAM229B",
  "gene": "UniProtKB:Q4G0N7",
  "term_label": "Unknown molecular function",
  "term_id": "UNKNOWN:0001",
  "gene_name": "Protein FAM229B"
}